{
  "gene_symbol": "C11orf86",
  "term_label": "Unknown cellular component",
  "term_id": "UNKNOWN:0003",
  "gene": "UniProtKB:A6NJI1",
  "gene_name": "Uncharacterized protein C11orf86"
}